{
  "term_id": "GO:0031507",
  "gene": "UniProtKB:O75530",
  "term_label": "heterochromatin formation",
  "gene_symbol": "EED",
  "gene_name": "Polycomb protein EED"
}